{
  "gene": "UniProtKB:Q8TEX9",
  "term_id": "GO:0005634",
  "gene_symbol": "IPO4",
  "gene_name": "Importin-4",
  "term_label": "nucleus"
}